{
  "gene": "UniProtKB:Q8NGA6",
  "gene_symbol": "OR10H5",
  "term_id": "GO:0005886",
  "term_label": "plasma membrane",
  "gene_name": "Olfactory receptor 10H5"
}